{
  "term_id": "GO:0086011",
  "term_label": "membrane repolarization during action potential",
  "gene_name": "Potassium voltage-gated channel subfamily E regulatory beta subunit 5",
  "gene": "UniProtKB:Q9UJ90",
  "gene_symbol": "KCNE5"
}